{
  "gene_symbol": "IP6K1",
  "gene_name": "Inositol hexakisphosphate kinase 1",
  "gene": "UniProtKB:Q92551",
  "term_id": "GO:0032958",
  "term_label": "inositol phosphate biosynthetic process"
}